{
  "term_id": "GO:0005737",
  "gene_name": "Ectoderm-neural cortex protein 1",
  "term_label": "cytoplasm",
  "gene_symbol": "ENC1",
  "gene": "UniProtKB:O14682"
}